regulation of wound healing, spreading of epidermal cells [GO:1903689] (biological process) Relationships: is a type of regulation of cell migration [GO:0030334]; is a type of regulation of wound healing [GO:0061041]; regulates GO:0035313 Subtypes: negative regulation of wound healing, spreading of epidermal cells [GO:1903690], GO:1903691 References: PMID:18394891 Sources: GOC:TermGenie, GOC:als, GO_REF:0000058 Definition: Any process that modulates the frequency, rate or extent of wound healing, spreading of epidermal cells.